{
  "gene_symbol": "ACSM2B",
  "gene_name": "Acyl-coenzyme A synthetase ACSM2B, mitochondrial",
  "gene": "UniProtKB:Q68CK6",
  "term_id": "GO:0015645",
  "term_label": "fatty acid ligase activity"
}